regulation of natural killer cell proliferation involved in immune response [GO:0032820] (biological process) Subtypes: negative regulation of natural killer cell proliferation involved in immune response [GO:0032821], positive regulation of natural killer cell proliferation involved in immune response [GO:0032822] Relationships: is a type of regulation of immune effector process [GO:0002697]; is a type of GO:0032817; is a type of regulation of immune response [GO:0050776]; RO_0002211 GO:0002324 Sources: GOC:mah Also known as: regulation of NK cell proliferation during immune response, regulation of natural killer cell proliferation during immune response Definition: Any process that modulates the frequency, rate or extent of natural killer cell proliferation as part of an immune response.